sinapate ester biosynthetic process [GO:0033525] (biological process) Sources: GOC:mah Relationships: is a type of phenylpropanoid biosynthetic process [GO:0009699]; is a type of phenol-containing compound biosynthetic process [GO:0046189] Definition: The chemical reactions and pathways resulting in the formation of ester derivates of sinapate, (2E)-3-(4-hydroxy-3,5-dimethoxyphenyl)prop-2-enoate. Also known as: sinapate ester anabolism, sinapate ester biosynthesis, sinapate ester formation, sinapate ester synthesis Regulation: regulated by regulation of sinapate ester biosynthetic process [GO:1903085]; negatively regulated by negative regulation of sinapate ester biosynthetic process [GO:1903086]